{
  "gene_symbol": "PPP3CC",
  "gene_name": "Serine_threonine-protein phosphatase 2B catalytic subunit gamma isoform",
  "gene": "UniProtKB:P48454",
  "term_label": "calmodulin-dependent protein phosphatase activity",
  "term_id": "GO:0033192"
}